positive regulation of retrograde protein transport, ER to cytosol [GO:1904154] (biological process) Definition: Any process that activates or increases the frequency, rate or extent of retrograde protein transport, ER to cytosol. Also known as: positive regulation of protein dislocation from ER, positive regulation of protein retrotranslocation from ER, positive regulation of retrograde protein transport, endoplasmic reticulum to cytosol, up regulation of protein dislocation from ER, up regulation of retrograde protein transport, ER to cytosol, up regulation of retrograde protein transport, endoplasmic reticulum to cytosol, up-regulation of protein dislocation from ER, up-regulation of protein retrotranslocation from ER, up-regulation of retrograde protein transport, ER to cytosol, up-regulation of retrograde protein transport, endoplasmic reticulum to cytosol, upregulation of protein dislocation from ER, upregulation of retrograde protein transport, ER to cytosol, upregulation of retrograde protein transport, endoplasmic reticulum to cytosol, activation of protein dislocation from ER, activation of retrograde protein transport, ER to cytosol, activation of retrograde protein transport, endoplasmic reticulum to cytosol Relationships: is a type of positive regulation of protein exit from endoplasmic reticulum [GO:0070863]; is a type of regulation of retrograde protein transport, ER to cytosol [GO:1904152]; positively regulates GO:0030970 References: PMID:18555783 Sources: GOC:PARL, GOC:TermGenie, GOC:bf, GO_REF:0000058